{
  "gene_symbol": "RFX4",
  "term_label": "DNA-binding transcription factor activity, RNA polymerase II-specific",
  "term_id": "GO:0000981",
  "gene": "UniProtKB:Q33E94",
  "gene_name": "Transcription factor RFX4"
}